{
  "term_id": "GO:0005739",
  "gene_symbol": "MICOS10",
  "gene_name": "MICOS complex subunit MIC10",
  "gene": "UniProtKB:Q5TGZ0",
  "term_label": "mitochondrion"
}